protein-DNA-RNA complex organization [GO:0001115] (biological process) Subtypes: protein-DNA-RNA complex assembly [GO:0001116], protein-DNA-RNA complex disassembly [GO:0001117], GO:0001119 Relationships: is a type of GO:0043933 Definition: Any process in which macromolecules aggregate, disaggregate, or are modified, resulting in the formation, disassembly, or alteration of a protein-DNA-RNA complex. Also known as: protein-DNA-RNA complex subunit organisation Sources: GOC:txnOH